{
  "gene_symbol": "FABP6",
  "gene_name": "Gastrotropin",
  "gene": "UniProtKB:P51161",
  "term_id": "GO:0005504",
  "term_label": "fatty acid binding"
}